root hair initiation [GO:0048766] (biological process) Relationships: is a type of GO:0000902; is part of root hair cell differentiation [GO:0048765] References: PMID:12468740 Sources: GOC:jid Definition: The process in which a protrusion or bulge is formed at the site of plant root hair outgrowth.